N-terminal protein formylation [GO:0018004] (biological process) Sources: GOC:ai Definition: The formylation of the N-terminal amino acid of proteins. Relationships: is a type of GO:0018256; is a type of N-terminal protein amino acid modification [GO:0031365]